{
  "gene": "UniProtKB:Q9H4B4",
  "term_label": "centrosome",
  "gene_symbol": "PLK3",
  "term_id": "GO:0005813",
  "gene_name": "Serine_threonine-protein kinase PLK3"
}